negative regulation of heart looping [GO:1901208] (biological process) Also known as: down regulation of cardiac looping, down regulation of heart looping, down-regulation of cardiac looping, down-regulation of heart looping, downregulation of cardiac looping, downregulation of heart looping, inhibition of cardiac looping, negative regulation of cardiac looping, inhibition of heart looping Definition: Any process that stops, prevents or reduces the frequency, rate or extent of heart looping. Relationships: is_a GO:1901207; is a type of negative regulation of morphogenesis of an epithelium [GO:1905331]; negatively regulates heart looping [GO:0001947] Sources: GOC:BHF, GOC:TermGenie